{
  "term_id": "GO:0001227",
  "term_label": "DNA-binding transcription repressor activity, RNA polymerase II-specific",
  "gene": "UniProtKB:Q05516",
  "gene_name": "Zinc finger and BTB domain-containing protein 16",
  "gene_symbol": "ZBTB16"
}